{
  "term_label": "forebrain development",
  "gene_name": "Paired box protein Pax-4",
  "term_id": "GO:0030900",
  "gene_symbol": "PAX4",
  "gene": "UniProtKB:O43316"
}